G protein-coupled neurotransmitter receptor activity involved in regulation of postsynaptic cytosolic calcium ion concentration [GO:0098872] (MF) Also known as: G-protein coupled neurotransmitter receptor activity involved in regulation of postsynaptic cytosolic calcium ion concentration, G-protein coupled neurotransmitter receptor activity involved in regulation of postsynaptic cytosolic calcium levels Definition: A G protein-coupled neurotransmitter receptor activity occurring in the postsynaptic membrane, that is involved in regulating the cytosolic concentration of calcium ions in the postsynapse. Sources: GOC:dos Relationships: is_a G protein-coupled neurotransmitter receptor activity [GO:0099528]; is a type of neurotransmitter receptor activity involved in regulation of postsynaptic cytosolic calcium ion concentration [GO:0099583]